{
  "gene": "UniProtKB:Q9NWS1",
  "gene_name": "PCNA-interacting partner",
  "term_label": "chromatin",
  "gene_symbol": "PARPBP",
  "term_id": "GO:0000785"
}